{
  "gene_name": "Myosin light chain kinase 2, skeletal_cardiac muscle",
  "gene": "UniProtKB:Q9H1R3",
  "term_label": "cardiac muscle tissue morphogenesis",
  "gene_symbol": "MYLK2",
  "term_id": "GO:0055008"
}